{
  "gene_symbol": "TRAJ41",
  "gene_name": "T cell receptor alpha joining 41 (Fragment)",
  "term_id": "UNKNOWN:0003",
  "term_label": "Unknown cellular component",
  "gene": "UniProtKB:A0A075B702"
}